uracil:monoatomic cation symporter activity [GO:0015505] (molecular function) Sources: GOC:mtg_transport Also known as: uracil:cation symporter activity, uracil permease activity Relationships: is a type of uracil transmembrane transporter activity [GO:0015210]; is a type of nucleobase:monoatomic cation symporter activity [GO:0015391] Definition: Enables the transfer of a solute or solutes from one side of a membrane to the other according to the reaction: uracil(out) + cation(out) = uracil(in) + cation(in).